positive regulation of mitotic spindle elongation (spindle phase three) [GO:0110164] (biological process) Relationships: is a type of positive regulation of mitotic spindle organization [GO:0110028]; is a type of regulation of mitotic spindle elongation (spindle phase three) [GO:0110162]; is a type of GO:1902846; positively regulates GO:0061805 References: PMID:27697865 Sources: GOC:vw Definition: Any process that activates or increases the frequency, rate or extent of the cell cycle process in which the distance is lengthened between poles of the mitotic spindle during mitotic anaphase B (spindle phase three).